tetrahydrobiopterin catabolic process [GO:0046147] (biological process) Relationships: is a type of diol catabolic process [GO:0034313]; is a type of pteridine-containing compound catabolic process [GO:0042560]; is a type of tetrahydrobiopterin metabolic process [GO:0046146] Definition: The chemical reactions and pathways resulting in the breakdown of tetrahydrobiopterin, the reduced form of biopterin (2-amino-4-hydroxy-6-(1,2-dihydroxypropyl)-pteridine). It functions as a hydroxylation coenzyme, e.g. in the conversion of phenylalanine to tyrosine. Sources: ISBN:0198506732 Also known as: 5,6,7,8-tetrahydrobiopterin catabolic process, tetrahydrobiopterin breakdown, tetrahydrobiopterin catabolism, tetrahydrobiopterin degradation